negative regulation of triglyceride transport [GO:1905884] (biological process) References: PMID:25849533 Sources: GOC:TermGenie, GO_REF:0000058 Definition: Any process that stops, prevents or reduces the frequency, rate or extent of triglyceride transport. Relationships: is a type of GO:1901507; is a type of GO:1905883; negatively regulates triglyceride transport [GO:0034197] Also known as: down regulation of triacylglycerol transport, down regulation of triglyceride transport, down-regulation of triacylglycerol transport, down-regulation of triglyceride transport, downregulation of triacylglycerol transport, downregulation of triglyceride transport, negative regulation of triacylglycerol transport, inhibition of triacylglycerol transport, inhibition of triglyceride transport